{
  "gene_name": "Chromatin assembly factor 1 subunit A",
  "gene_symbol": "CHAF1A",
  "gene": "UniProtKB:Q13111",
  "term_id": "GO:0033186",
  "term_label": "CAF-1 complex"
}